{
  "term_id": "GO:0051893",
  "term_label": "regulation of focal adhesion assembly",
  "gene": "UniProtKB:Q9UPQ0",
  "gene_name": "LIM and calponin homology domains-containing protein 1",
  "gene_symbol": "LIMCH1"
}